{
  "term_id": "GO:0015459",
  "gene_name": "Potassium voltage-gated channel subfamily B member 2",
  "gene": "UniProtKB:Q92953",
  "term_label": "potassium channel regulator activity",
  "gene_symbol": "KCNB2"
}